{
  "gene_name": "Heat shock factor protein 4",
  "term_id": "GO:0005634",
  "gene_symbol": "HSF4",
  "gene": "UniProtKB:Q9ULV5",
  "term_label": "nucleus"
}